{
  "gene": "UniProtKB:A6NM43",
  "gene_symbol": "CCT8L1P",
  "term_label": "protein folding",
  "gene_name": "Putative T-complex protein 1 subunit theta-like 1",
  "term_id": "GO:0006457"
}